{
  "term_id": "GO:0004252",
  "gene_symbol": "CTRC",
  "term_label": "serine-type endopeptidase activity",
  "gene_name": "Chymotrypsin-C",
  "gene": "UniProtKB:Q99895"
}